receptor localization to non-motile cilium [GO:0097500] (biological process) Also known as: receptor localization to nonmotile primary cilium Relationships: is a type of GO:0097499; is_a protein localization to ciliary membrane [GO:1903441] References: PMID:23128241 Sources: GOC:cilia, GOC:kmv Definition: A process in which a receptor is transported to, or maintained in, a location within a non-motile cilium.